{
  "term_label": "pyrroline-5-carboxylate reductase activity",
  "gene": "UniProtKB:Q6NXP6",
  "gene_symbol": "NOXRED1",
  "gene_name": "NADP-dependent oxidoreductase domain-containing protein 1",
  "term_id": "GO:0004735"
}